{
  "gene_name": "C-C chemokine receptor type 6",
  "gene_symbol": "CCR6",
  "gene": "UniProtKB:P51684",
  "term_label": "positive regulation of dendritic cell chemotaxis",
  "term_id": "GO:2000510"
}